Hsp90 protein binding [GO:0051879] (molecular function) Relationships: is a type of heat shock protein binding [GO:0031072] Definition: Binding to Hsp90 proteins, any of a group of heat shock proteins around 90kDa in size. Also known as: Hsp90 binding, Hsp90 class protein binding Sources: GOC:ai